{
  "term_id": "GO:0005886",
  "gene_name": "Olfactory receptor 2J2",
  "gene": "UniProtKB:O76002",
  "gene_symbol": "OR2J2",
  "term_label": "plasma membrane"
}